{
  "term_label": "cell migration",
  "term_id": "GO:0016477",
  "gene_name": "Cadherin-22",
  "gene": "UniProtKB:Q9UJ99",
  "gene_symbol": "CDH22"
}